{
  "term_label": "Unknown biological process",
  "gene": "UniProtKB:Q12894",
  "gene_name": "Interferon-related developmental regulator 2",
  "gene_symbol": "IFRD2",
  "term_id": "UNKNOWN:0002"
}